{
  "gene": "UniProtKB:Q7Z5R6",
  "term_label": "plasma membrane",
  "gene_name": "Amyloid beta A4 precursor protein-binding family B member 1-interacting protein",
  "term_id": "GO:0005886",
  "gene_symbol": "APBB1IP"
}